{
  "gene": "UniProtKB:Q30KQ6",
  "term_id": "GO:0060326",
  "gene_name": "Beta-defensin 114",
  "term_label": "cell chemotaxis",
  "gene_symbol": "DEFB114"
}